micromitophagy [GO:0000424] (biological process) Note: Note that this term is not a child of mitophagy because the community generally uses the latter to refer to the macroautophagy of mitochondria. Relationships: is a type of autophagy of mitochondrion [GO:0000422]; is_a GO:0016237 References: PMID:15798367, PMID:27003723 Definition: Degradation of a mitochondrion by microautophagy.